{
  "gene_name": "Keratin-associated protein 10-7",
  "gene": "UniProtKB:P60409",
  "term_id": "UNKNOWN:0003",
  "term_label": "Unknown cellular component",
  "gene_symbol": "KRTAP10-7"
}